L-proline betaine biosynthetic process [GO:0019503] (BP) References: PMID:14367364 Sources: GOC:ai Definition: The chemical reactions and pathways resulting in the formation of stachydrine, N-methylproline methylbetaine, the betaine derivative of L-proline. Relationships: is a type of amino-acid betaine biosynthetic process [GO:0006578]; is a type of alkaloid biosynthetic process [GO:0009821]; is a type of L-amino acid biosynthetic process [GO:0170034]; is a type of GO:0170043 Also known as: stachydrine anabolism, stachydrine biosynthesis, stachydrine biosynthetic process, stachydrine formation, stachydrine synthesis